neural crest formation [GO:0014029] (biological process) Relationships: is a type of epithelial to mesenchymal transition [GO:0001837]; is_a anatomical structure formation involved in morphogenesis [GO:0048646]; is part of chordate embryonic development [GO:0043009] Definition: The formation of the specialized region of ectoderm between the neural ectoderm (neural plate) and non-neural ectoderm. The neural crest gives rise to the neural crest cells that migrate away from this region as neural tube formation proceeds. Sources: GOC:dh, GOC:ef Regulation: regulated by GO:0090299; RO_0002213 by GO:0090300; negatively regulated by GO:0090301